{
  "term_label": "actin polymerization or depolymerization",
  "gene_symbol": "CAPG",
  "gene": "UniProtKB:P40121",
  "gene_name": "Macrophage-capping protein",
  "term_id": "GO:0008154"
}